{
  "gene_symbol": "DTNBP1",
  "term_id": "GO:0030672",
  "term_label": "synaptic vesicle membrane",
  "gene": "UniProtKB:Q96EV8",
  "gene_name": "Dysbindin"
}